heteroduplex DNA loop binding [GO:0000404] (molecular function) Definition: Binding to a DNA segment containing a loop. A loop occurs when DNA contains a large insertion or deletion that causes a region of unpaired single-stranded DNA to loop out, while the rest of the DNA is in a paired double-stranded configuration. Relationships: is a type of DNA secondary structure binding [GO:0000217]; is a type of DNA insertion or deletion binding [GO:0032135] Also known as: loop DNA binding References: PMID:16781730 Sources: GOC:elh